regulation of plasma lipoprotein particle levels [GO:0097006] (biological process) Also known as: plasma lipoprotein particle homeostasis Sources: GOC:BHF Relationships: is a type of regulation of biological process [GO:0050789] Definition: Any process involved in the maintenance of internal levels of plasma lipoprotein particles within an organism.